{
  "gene": "UniProtKB:P78411",
  "gene_name": "Iroquois-class homeodomain protein IRX-5",
  "term_label": "DNA-binding transcription factor activity, RNA polymerase II-specific",
  "gene_symbol": "IRX5",
  "term_id": "GO:0000981"
}